{
  "term_label": "ADP-ribose diphosphatase activity",
  "gene": "UniProtKB:Q3LIE5",
  "gene_symbol": "ADPRM",
  "term_id": "GO:0047631",
  "gene_name": "Manganese-dependent ADP-ribose_CDP-alcohol diphosphatase"
}